negative regulation of penicillin biosynthetic process [GO:1900197] (biological process) Sources: GOC:TermGenie, GOC:di Definition: Any process that stops, prevents or reduces the frequency, rate or extent of penicillin biosynthetic process. Also known as: down regulation of penicillin anabolism, down regulation of penicillin biosynthesis, down regulation of penicillin biosynthetic process, down regulation of penicillin formation, down regulation of penicillin synthesis, down-regulation of penicillin anabolism, down-regulation of penicillin biosynthesis, down-regulation of penicillin biosynthetic process, down-regulation of penicillin formation, down-regulation of penicillin synthesis, downregulation of penicillin anabolism, downregulation of penicillin biosynthesis, downregulation of penicillin biosynthetic process, downregulation of penicillin formation, downregulation of penicillin synthesis, inhibition of penicillin anabolism, inhibition of penicillin biosynthesis, inhibition of penicillin formation, inhibition of penicillin synthesis, negative regulation of penicillin anabolism, negative regulation of penicillin biosynthesis, negative regulation of penicillin formation, negative regulation of penicillin synthesis, inhibition of penicillin biosynthetic process Relationships: is_a negative regulation of amide metabolic process [GO:0034249]; is a type of negative regulation of small molecule metabolic process [GO:0062014]; is a type of regulation of penicillin biosynthetic process [GO:1900196]; is a type of negative regulation of secondary metabolite biosynthetic process [GO:1900377]; RO_0002212 penicillin biosynthetic process [GO:0042318]